{
  "gene_name": "Zinc finger CCCH domain-containing protein 6",
  "gene": "UniProtKB:P61129",
  "term_label": "negative regulation of DNA-templated transcription, elongation",
  "gene_symbol": "ZC3H6",
  "term_id": "GO:0032785"
}